regulation of water channel activity [GO:1902427] (biological process) Relationships: is a type of regulation of transmembrane transporter activity [GO:0022898]; regulates water channel activity [GO:0015250] References: PMID:22095752 Sources: GOC:TermGenie, GOC:nhn Definition: Any process that modulates the frequency, rate or extent of water channel activity. Also known as: regulation of aquaporin, regulation of aquaporin permeability